{
  "gene": "UniProtKB:Q12908",
  "term_id": "GO:0016324",
  "gene_symbol": "SLC10A2",
  "term_label": "apical plasma membrane",
  "gene_name": "Ileal sodium_bile acid cotransporter"
}